{
  "gene_symbol": "PRKRIP1",
  "gene": "UniProtKB:Q9H875",
  "term_label": "protein kinase inhibitor activity",
  "gene_name": "PRKR-interacting protein 1",
  "term_id": "GO:0004860"
}